{
  "gene": "UniProtKB:Q9HCG1",
  "term_id": "GO:0006357",
  "gene_name": "Zinc finger protein 160",
  "term_label": "regulation of transcription by RNA polymerase II",
  "gene_symbol": "ZNF160"
}